{
  "term_id": "GO:0006865",
  "gene_symbol": "SLC6A12",
  "gene_name": "Sodium- and chloride-dependent betaine transporter",
  "term_label": "amino acid transport",
  "gene": "UniProtKB:P48065"
}